{
  "gene": "UniProtKB:Q15149",
  "term_label": "structural constituent of cytoskeleton",
  "gene_symbol": "PLEC",
  "term_id": "GO:0005200",
  "gene_name": "Plectin"
}